kynurenic acid metabolic process [GO:0034275] (biological process) Sources: GOC:mah Relationships: is a type of monocarboxylic acid metabolic process [GO:0032787] Also known as: 4-hydroxyquinoline-2-carboxylic acid metabolic process, kynurenic acid metabolism Definition: The chemical reactions and pathways involving kynurenic acid, 4-hydroxyquinoline-2-carboxylic acid. Subtypes: kynurenic acid biosynthetic process [GO:0034276]